regulation of calcium-independent cell-cell adhesion [GO:0051040] (biological process) Sources: GOC:ai Definition: Any process that modulates the frequency, rate or extent of the attachment of one cell to another cell via adhesion molecules that do not require the presence of calcium for the interaction. Subtypes: GO:0051041, negative regulation of calcium-independent cell-cell adhesion [GO:0051042] Relationships: is a type of GO:0022407; regulates calcium-independent cell-cell adhesion [GO:0016338]